{
  "term_id": "GO:0044233",
  "gene_symbol": "TMX2",
  "gene_name": "Thioredoxin-related transmembrane protein 2",
  "term_label": "mitochondria-associated endoplasmic reticulum membrane contact site",
  "gene": "UniProtKB:Q9Y320"
}